cell cycle DNA replication maintenance of fidelity [GO:1902298] (biological process) Definition: Any maintenance of fidelity that is involved in cell cycle DNA replication. Also known as: maintenance of fidelity involved in cell cycle DNA replication, maintenance of fidelity during DNA-dependent DNA replication involved in cell cycle DNA replication Sources: GOC:TermGenie, GOC:mtg_cell_cycle Subtypes: mitotic DNA replication maintenance of fidelity [GO:1990505] Relationships: is a type of cell cycle process [GO:0022402]; is a type of GO:0045005; is part of GO:0044786